{
  "gene": "UniProtKB:O75593",
  "term_label": "positive regulation of transcription by RNA polymerase II",
  "gene_name": "Forkhead box protein H1",
  "term_id": "GO:0045944",
  "gene_symbol": "FOXH1"
}